body fluid secretion [GO:0007589] (BP) Relationships: is a type of secretion [GO:0046903]; is a type of regulation of body fluid levels [GO:0050878] Sources: GOC:ai, GOC:dph, GOC:mah, GOC:tb Subtypes: lactation [GO:0007595], pancreatic juice secretion [GO:0030157], cerebrospinal fluid secretion [GO:0033326], saliva secretion [GO:0046541], milk ejection reflex [GO:0060156], tear secretion [GO:0070075], mucus secretion [GO:0070254], sweat secretion [GO:0160269] Definition: The controlled release of a fluid by a cell or tissue in an animal.